{
  "gene_name": "Type III endosome membrane protein TEMP",
  "gene": "UniProtKB:Q8IVY1",
  "term_label": "Unknown cellular component",
  "term_id": "UNKNOWN:0003",
  "gene_symbol": "C1orf210"
}